{
  "gene_symbol": "DUX4L9",
  "term_id": "GO:0006357",
  "gene_name": "Double homeobox protein 4C",
  "term_label": "regulation of transcription by RNA polymerase II",
  "gene": "UniProtKB:Q6RFH8"
}